{
  "term_label": "cytoplasmic vesicle",
  "term_id": "GO:0031410",
  "gene_name": "Trafficking kinesin-binding protein 2",
  "gene_symbol": "TRAK2",
  "gene": "UniProtKB:O60296"
}